lymphocyte chemotaxis [GO:0048247] (biological process) Regulation: positively regulated by positive regulation of lymphocyte chemotaxis [GO:0140131]; RO_0002211 by regulation of lymphocyte chemotaxis [GO:1901623]; negatively regulated by negative regulation of lymphocyte chemotaxis [GO:1901624] Definition: The directed movement of a lymphocyte in response to an external stimulus. Relationships: is a type of leukocyte chemotaxis [GO:0030595]; is a type of GO:0072676 Subtypes: GO:0002518, T cell chemotaxis [GO:0010818], GO:0035747, B cell chemotaxis [GO:0035754] References: PMID:12391252 Sources: GOC:hjd, GOC:jid